{
  "gene_name": "XK-related protein 6",
  "gene_symbol": "XKR6",
  "gene": "UniProtKB:Q5GH73",
  "term_id": "GO:0043652",
  "term_label": "engulfment of apoptotic cell"
}